migration in host [GO:0044001] (biological process) Also known as: migration within host Definition: The directional movement of an organism from one place to another within its host organism. The host is defined as the larger of the organisms involved in a symbiotic interaction. Subtypes: transport of virus in multicellular host [GO:0046739], GO:0106259, symbiont-mediated migration across host tissue barrier [GO:0141142] Relationships: is a type of GO:0051701 Sources: GOC:cc